cellular response to immobilization stress [GO:0035903] (biological process) Relationships: is a type of GO:0033554; is a type of response to immobilization stress [GO:0035902] Also known as: cellular response to immobilisation stress, cellular response to restraint stress References: PMID:17683801, PMID:19893991 Sources: GOC:bf Definition: Any process that results in a change in state or activity of a cell (in terms of movement, secretion, enzyme production, gene expression, etc.) as a result of being rendered immobile.